{
  "term_label": "endoplasmic reticulum membrane",
  "gene": "UniProtKB:Q9Y6I9",
  "gene_symbol": "TEX264",
  "term_id": "GO:0005789",
  "gene_name": "Testis-expressed protein 264"
}